optic vesicle elongation [GO:0003405] (biological process) Definition: The developmental growth that results in the lengthening of the optic vesicle in the posterior direction. Relationships: is_a developmental growth involved in morphogenesis [GO:0060560]; is part of optic vesicle morphogenesis [GO:0003404] Sources: GOC:ascb_2009, GOC:dph, GOC:tb